{
  "term_label": "RNA binding",
  "gene_name": "RNA-binding protein 10",
  "gene": "UniProtKB:P98175",
  "term_id": "GO:0003723",
  "gene_symbol": "RBM10"
}